{
  "term_label": "ribonucleoprotein complex",
  "term_id": "GO:1990904",
  "gene": "UniProtKB:Q9H6T0",
  "gene_symbol": "ESRP2",
  "gene_name": "Epithelial splicing regulatory protein 2"
}